{
  "gene": "UniProtKB:Q15554",
  "gene_name": "Telomeric repeat-binding factor 2",
  "term_id": "GO:0070187",
  "term_label": "shelterin complex",
  "gene_symbol": "TERF2"
}